perichromatin fibrils [GO:0005726] (cellular component) Relationships: is a type of GO:0110165; is part of nuclear chromosome [GO:0000228]; is part of chromatin [GO:0000785] References: PMID:14731598 Definition: Structures of variable diameter visible in the nucleoplasm by electron microscopy, mainly observed near the border of condensed chromatin. The fibrils are enriched in RNA, and are believed to be sites of pre-mRNA splicing and polyadenylylation representing the in situ form of nascent transcripts.